antigen processing and presentation, endogenous lipid antigen via MHC class Ib [GO:0048006] (biological process) Relationships: is a type of antigen processing and presentation of endogenous antigen [GO:0019883]; is a type of GO:0048003 Definition: The process in which an antigen-presenting cell expresses lipid antigen of endogenous origin in association with an MHC class Ib protein complex on its cell surface. Class Ib here refers to non-classical class I molecules, such as those of the CD1 family. References: PMID:10375559, PMID:15928678, PMID:15928680 Sources: GOC:add Also known as: antigen presentation, endogenous lipid antigen, endogenous lipid antigen processing and presentation via MHC class Ib